3'-tRNA processing endoribonuclease activity [GO:0042781] (molecular function) References: PMID:12032089, PMID:21208191 Sources: EC:3.1.26.11 Definition: Catalysis of the endonucleolytic cleavage of RNA, removing extra 3' nucleotides from tRNA precursor, generating 3' termini of tRNAs. A 3'-hydroxy group is left at the tRNA terminus and a 5'-phosphoryl group is left at the trailer molecule. Relationships: is a type of tRNA-specific ribonuclease activity [GO:0004549]; is a type of GO:0016891; is part of tRNA 3'-end processing [GO:0042780] Also known as: RNase Z activity, ribonuclease Z activity, 3' tRNA processing endoribonuclease activity, 3' tRNase activity, tRNA 3' endonuclease activity, 3 tRNase activity, tRNA 3 endonuclease activity, tRNAse Z